apoptotic process involved in endocardial cushion morphogenesis [GO:0003277] (biological process) Sources: GOC:mtg_apoptosis, GOC:mtg_heart Relationships: is a type of apoptotic process involved in heart morphogenesis [GO:0003278]; is part of GO:0003203 Also known as: apoptosis involved in endocardial cushion morphogenesis Definition: Any apoptotic process that contributes to the shaping of an endocardial cushion. The endocardial cushion is a specialized region of mesenchymal cells that will give rise to the heart septa and valves.